{
  "gene": "UniProtKB:Q9NZP2",
  "gene_symbol": "OR6C2",
  "term_label": "Unknown biological process",
  "term_id": "UNKNOWN:0002",
  "gene_name": "Olfactory receptor 6C2"
}